{
  "gene_name": "Peroxisomal biogenesis factor 3",
  "term_label": "protein import into peroxisome membrane",
  "term_id": "GO:0045046",
  "gene": "UniProtKB:P56589",
  "gene_symbol": "PEX3"
}